{
  "term_id": "GO:0006508",
  "gene": "UniProtKB:Q8N4T0",
  "gene_symbol": "CPA6",
  "gene_name": "Carboxypeptidase A6",
  "term_label": "proteolysis"
}